fatty acid oxidation [GO:0019395] (biological process) Relationships: is a type of fatty acid metabolic process [GO:0006631]; is a type of lipid oxidation [GO:0034440] Subtypes: fatty acid alpha-oxidation [GO:0001561], fatty acid beta-oxidation [GO:0006635], fatty acid omega-oxidation [GO:0010430] Sources: ISBN:0198506732 Regulation: regulated by GO:0046320; positively regulated by positive regulation of fatty acid oxidation [GO:0046321]; negatively regulated by negative regulation of fatty acid oxidation [GO:0046322] Definition: The removal of one or more electrons from a fatty acid, with or without the concomitant removal of a proton or protons, by reaction with an electron-accepting substance, by addition of oxygen or by removal of hydrogen.